{
  "gene_name": "Transcription factor SOX-12",
  "term_id": "GO:0030182",
  "gene": "UniProtKB:O15370",
  "gene_symbol": "SOX12",
  "term_label": "neuron differentiation"
}